negative regulation of mesenchymal cell apoptotic process involved in metanephros development [GO:1900212] (biological process) Also known as: down regulation of mesenchymal cell apoptosis involved in metanephros development, down-regulation of mesenchymal cell apoptosis involved in metanephros development, downregulation of mesenchymal cell apoptosis involved in metanephros development, inhibition of mesenchymal cell apoptosis involved in metanephros development, negative regulation of mesenchymal cell apoptosis involved in metanephros development Subtypes: negative regulation of mesenchymal cell apoptotic process involved in metanephric nephron morphogenesis [GO:0072305] References: PMID:17314325 Sources: GOC:TermGenie, GOC:mtg_apoptosis, GOC:mtg_kidney_jan10, GOC:yaf Relationships: is a type of regulation of mesenchymal cell apoptotic process involved in metanephros development [GO:1900211]; is_a negative regulation of apoptotic process involved in development [GO:1904746]; is a type of negative regulation of mesenchymal cell apoptotic process [GO:2001054]; negatively regulates GO:1900200 Definition: Any process that stops, prevents or reduces the frequency, rate or extent of mesenchymal cell apoptotic process involved in metanephros development.